positive regulation of leukocyte differentiation [GO:1902107] (biological process) Subtypes: positive regulation of myeloid leukocyte differentiation [GO:0002763], positive regulation of lymphocyte differentiation [GO:0045621], positive regulation of dendritic cell differentiation [GO:2001200] Definition: Any process that activates or increases the frequency, rate or extent of leukocyte differentiation. Sources: GOC:TermGenie, GOC:add Also known as: positive regulation of immune cell differentiation, positive regulation of leucocyte differentiation, up regulation of immune cell differentiation, up regulation of leucocyte differentiation, up regulation of leukocyte differentiation, up-regulation of immune cell differentiation, up-regulation of leucocyte differentiation, up-regulation of leukocyte differentiation, upregulation of immune cell differentiation, upregulation of leucocyte differentiation, upregulation of leukocyte differentiation, activation of immune cell differentiation, activation of leucocyte differentiation, activation of leukocyte differentiation Relationships: is a type of regulation of leukocyte differentiation [GO:1902105]; is a type of positive regulation of hemopoiesis [GO:1903708]; RO_0002213 GO:0002521